{
  "gene_symbol": "CHMP2A",
  "term_label": "protein transport",
  "term_id": "GO:0015031",
  "gene": "UniProtKB:O43633",
  "gene_name": "Charged multivesicular body protein 2a"
}